mesonephric proximal tubule morphogenesis [GO:0061276] (biological process) Definition: The process in which the anatomical structures of a mesonephric proximal tubule are generated and organized. The mesonephric proximal tubule extends from the capsule to the distal tubule. Relationships: is a type of GO:0061240; is a type of proximal tubule morphogenesis [GO:0072158]; is part of mesonephric proximal tubule development [GO:0061275] Sources: GOC:mtg_kidney_jan10